{
  "term_label": "regulation of DNA-templated transcription",
  "term_id": "GO:0006355",
  "gene": "UniProtKB:A6NK75",
  "gene_name": "Zinc finger protein 98",
  "gene_symbol": "ZNF98"
}